ammonium homeostasis [GO:0097272] (biological process) Also known as: ammonia homeostasis Subtypes: intracellular ammonium homeostasis [GO:0097275] Definition: Any biological process involved in the maintenance of an internal steady state of ammonium. References: PMID:12695560 Sources: GOC:yaf Relationships: is a type of inorganic ion homeostasis [GO:0098771]